{
  "gene_symbol": "XRCC3",
  "term_id": "GO:0071140",
  "term_label": "resolution of mitotic recombination intermediates",
  "gene_name": "DNA repair protein XRCC3",
  "gene": "UniProtKB:O43542"
}